{
  "gene_symbol": "TRBV2",
  "gene_name": "T cell receptor beta variable 2",
  "gene": "UniProtKB:A0A1B0GX68",
  "term_id": "GO:0005886",
  "term_label": "plasma membrane"
}